RNA ligase activity [GO:0008452] (MF) Sources: GOC:mah Subtypes: RNA ligase (ATP) activity [GO:0003972], RNA ligase (GTP) activity [GO:0170057] Definition: Catalysis of the formation of a phosphodiester bond between a hydroxyl group at the end of one RNA chain and the phosphate group at the end of another. Relationships: is_a ligase activity, forming phosphoric ester bonds [GO:0016886]; is a type of catalytic activity, acting on RNA [GO:0140098]